positive regulation of pentadecane biosynthetic process [GO:1900889] (biological process) Also known as: up regulation of pentadecane biosynthetic process, up-regulation of pentadecane biosynthetic process, upregulation of pentadecane biosynthetic process, activation of pentadecane anabolism, activation of pentadecane biosynthesis, activation of pentadecane biosynthetic process, activation of pentadecane formation, activation of pentadecane synthesis, positive regulation of pentadecane anabolism, positive regulation of pentadecane biosynthesis, positive regulation of pentadecane formation, positive regulation of pentadecane synthesis, up regulation of pentadecane anabolism, up regulation of pentadecane biosynthesis, up regulation of pentadecane formation, up regulation of pentadecane synthesis, up-regulation of pentadecane anabolism, up-regulation of pentadecane biosynthesis, up-regulation of pentadecane formation, up-regulation of pentadecane synthesis, upregulation of pentadecane anabolism, upregulation of pentadecane biosynthesis, upregulation of pentadecane formation, upregulation of pentadecane synthesis Relationships: is a type of GO:1900887; is a type of positive regulation of alkane biosynthetic process [GO:1901579]; RO_0002213 pentadecane biosynthetic process [GO:1900634] Definition: Any process that activates or increases the frequency, rate or extent of pentadecane biosynthetic process. Sources: GOC:TermGenie, GOC:mengo_curators